{
  "term_label": "extracellular space",
  "gene": "UniProtKB:P26022",
  "term_id": "GO:0005615",
  "gene_name": "Pentraxin-related protein PTX3",
  "gene_symbol": "PTX3"
}